positive regulation of phosphorus metabolic process [GO:0010562] (biological process) Subtypes: positive regulation of phosphate metabolic process [GO:0045937], positive regulation of phosphorus utilization [GO:0045949], GO:1900976 Definition: Any process that increases the frequency, rate or extent of the chemical reactions and pathways involving phosphorus or compounds containing phosphorus. Sources: GOC:dph, GOC:tb Relationships: is a type of positive regulation of metabolic process [GO:0009893]; is a type of GO:0051174; positively regulates phosphorus metabolic process [GO:0006793]